{
  "gene_name": "Ubiquitin_ISG15-conjugating enzyme E2 L6",
  "term_label": "ubiquitin conjugating enzyme activity",
  "term_id": "GO:0061631",
  "gene": "UniProtKB:O14933",
  "gene_symbol": "UBE2L6"
}